{
  "gene": "UniProtKB:O75554",
  "term_label": "RNA binding",
  "gene_name": "WW domain-binding protein 4",
  "term_id": "GO:0003723",
  "gene_symbol": "WBP4"
}